{
  "gene_symbol": "SRR",
  "gene": "UniProtKB:Q9GZT4",
  "term_id": "GO:0003941",
  "term_label": "L-serine ammonia-lyase activity",
  "gene_name": "Serine racemase"
}